UDP-glucose 4,6-dehydratase activity [GO:0050377] (molecular function) Also known as: UDP-D-glucose oxidoreductase activity, UDP-D-glucose-4,6-hydrolyase activity, UDP-glucose 4,6-hydro-lyase (UDP-4-dehydro-6-deoxy-D-glucose-forming), UDP-glucose 4,6-hydro-lyase activity, UDPglucose 4,6-dehydratase activity, UDPglucose 4,6-hydro-lyase activity Definition: Catalysis of the reaction: UDP-D-glucose = H2O + UDP-4-dehydro-6-deoxy-D-glucose. Relationships: is a type of GO:0016836 Sources: EC:4.2.1.76, RHEA:21500